U2-type precatalytic spliceosome [GO:0071005] (cellular component) Definition: A spliceosomal complex that is formed by the recruitment of the preassembled U4/U6.U5 tri-snRNP to the prespliceosome. Although all 5 snRNPs are present, the precatalytic spliceosome is catalytically inactive. The precatalytic spliceosome includes many proteins in addition to those found in the U1, U2 and U4/U6.U5 snRNPs. Relationships: is a type of U2-type spliceosomal complex [GO:0005684]; is a type of precatalytic spliceosome [GO:0071011]; BFO_0000051 U1 snRNP [GO:0005685]; BFO_0000051 U2 snRNP [GO:0005686]; has part U4/U6 x U5 tri-snRNP complex [GO:0046540] Also known as: major precatalytic spliceosome, GT-AG precatalytic spliceosome, mammalian U2-type spliceosomal complex B, mammalian U2-type spliceosomal complex B1, yeast U12-type spliceosomal complex A2-1 References: PMID:18322460, PMID:19239890 Sources: GOC:ab, GOC:krc, GOC:mah